nuclear envelope budding [GO:0140591] (biological process) References: PMID:27236823, PMID:32503943 Relationships: is_a GO:0051168 Definition: The process by which large macromolecular complexes are budded through the inner nuclear membrane, into the perinuclear space, thus acquiring a membrane envelope. The enveloped particle fuses with the outer nuclear membrane and is released into the cytoplasm.